{
  "gene": "UniProtKB:Q6UXG2",
  "term_label": "Unknown molecular function",
  "gene_symbol": "ELAPOR1",
  "gene_name": "Endosome_lysosome-associated apoptosis and autophagy regulator 1",
  "term_id": "UNKNOWN:0001"
}